ureter smooth muscle development [GO:0072191] (biological process) Definition: The process whose specific outcome is the progression of smooth muscle in the ureter over time, from its formation to the mature structure. Relationships: is a type of smooth muscle tissue development [GO:0048745]; is part of ureter development [GO:0072189] Sources: GOC:mtg_kidney_jan10